{
  "term_id": "GO:0000333",
  "gene_symbol": "TERT",
  "term_label": "telomerase catalytic core complex",
  "gene_name": "Telomerase reverse transcriptase",
  "gene": "UniProtKB:O14746"
}